{
  "term_label": "phospholipid dephosphorylation",
  "gene": "UniProtKB:Q32ZL2",
  "gene_name": "Phospholipid phosphatase-related protein type 5",
  "gene_symbol": "PLPPR5",
  "term_id": "GO:0046839"
}